{
  "gene_name": "UDP-glucose 4-epimerase",
  "term_label": "UDP-glucose 4-epimerase activity",
  "term_id": "GO:0003978",
  "gene": "UniProtKB:Q14376",
  "gene_symbol": "GALE"
}